{
  "gene_name": "116 kDa U5 small nuclear ribonucleoprotein component",
  "gene": "UniProtKB:Q15029",
  "term_id": "GO:0003924",
  "term_label": "GTPase activity",
  "gene_symbol": "EFTUD2"
}